{
  "term_id": "GO:0005634",
  "gene": "UniProtKB:Q96K75",
  "gene_name": "Zinc finger protein 514",
  "gene_symbol": "ZNF514",
  "term_label": "nucleus"
}